cell hair [GO:0070451] (CC) Relationships: is a type of plasma membrane bounded cell projection [GO:0120025] Definition: A long, thin cell projection that contains F-actin and tubulin, with microtubules centrally located and F-actin peripherally located. Also known as: non-sensory hair, imaginal disc-derived wing hair References: PMID:11526084